{
  "term_label": "GDP-mannose biosynthetic process",
  "gene_name": "Mannose-6-phosphate isomerase",
  "term_id": "GO:0009298",
  "gene": "UniProtKB:P34949",
  "gene_symbol": "MPI"
}